{
  "gene_symbol": "STPG1",
  "term_id": "UNKNOWN:0001",
  "term_label": "Unknown molecular function",
  "gene_name": "O(6)-methylguanine-induced apoptosis 2",
  "gene": "UniProtKB:Q5TH74"
}